{
  "term_id": "GO:0038023",
  "gene": "UniProtKB:Q9H3W5",
  "gene_name": "Leucine-rich repeat neuronal protein 3",
  "gene_symbol": "LRRN3",
  "term_label": "signaling receptor activity"
}